{
  "gene_name": "GTP-binding protein REM 2",
  "gene_symbol": "REM2",
  "gene": "UniProtKB:Q8IYK8",
  "term_label": "GTP binding",
  "term_id": "GO:0005525"
}